regulation of interleukin-20 production [GO:0032664] (biological process) Also known as: regulation of IL-20 production, regulation of interleukin-20 biosynthetic process Definition: Any process that modulates the frequency, rate, or extent of interleukin-20 production. Sources: GOC:mah Relationships: is a type of regulation of cytokine production [GO:0001817]; regulates GO:0032624 Subtypes: negative regulation of interleukin-20 production [GO:0032704], positive regulation of interleukin-20 production [GO:0032744]